exocyst [GO:0000145] (cellular component) References: PMID:15292201, PMID:27243008, PMID:9700152 Sources: GOC:cilia Definition: A protein complex peripherally associated with the plasma membrane that determines where vesicles dock and fuse. At least eight complex components are conserved between yeast and mammals. Relationships: is a type of vesicle tethering complex [GO:0099023]; is part of cell cortex [GO:0005938] Also known as: Sec6/8 complex, exocyst complex